sensory perception of high humidity [GO:0098510] (biological process) References: PMID:18269908 Relationships: is a type of sensory perception of humidity [GO:0098509] Definition: The series of events required for an organism to detect high environmental humidity, convert this detection into a molecular signal, and recognize and characterize the signal. This is a neurological process.